{
  "gene_symbol": "PLAAT2",
  "term_label": "N-acylphosphatidylethanolamine metabolic process",
  "gene": "UniProtKB:Q9NWW9",
  "gene_name": "Phospholipase A and acyltransferase 2",
  "term_id": "GO:0070292"
}